{
  "term_label": "general transcription initiation factor activity",
  "gene_symbol": "TBPL1",
  "gene": "UniProtKB:P62380",
  "term_id": "GO:0140223",
  "gene_name": "TATA box-binding protein-like 1"
}